{
  "term_label": "serine-type endopeptidase inhibitor activity",
  "gene_name": "Serpin B7",
  "term_id": "GO:0004867",
  "gene_symbol": "SERPINB7",
  "gene": "UniProtKB:O75635"
}